{
  "gene_name": "Immunoglobulin heavy variable 3-30-3",
  "term_label": "Unknown cellular component",
  "gene_symbol": "IGHV3-30-3",
  "term_id": "UNKNOWN:0003",
  "gene": "UniProtKB:P0DP02"
}